negative regulation of interleukin-25 production [GO:0032709] (biological process) Definition: Any process that stops, prevents, or reduces the frequency, rate, or extent of interleukin-25 production. Sources: GOC:mah Relationships: is a type of negative regulation of cytokine production [GO:0001818]; is a type of GO:0032669; negatively regulates interleukin-25 production [GO:0032629] Also known as: down regulation of interleukin-25 production, down-regulation of interleukin-25 production, downregulation of interleukin-25 production, negative regulation of IL-25 production, inhibition of interleukin-25 production, negative regulation of interleukin-25 biosynthetic process, negative regulation of interleukin-25 secretion